relaxation of vascular associated smooth muscle [GO:0060087] (BP) References: PMID:15867178, PMID:19996365, PMID:27389411 Sources: GOC:BHF, GOC:BHF_miRNA, GOC:TermGenie, GOC:dph, GOC:rph Relationships: is a type of relaxation of smooth muscle [GO:0044557]; is a type of negative regulation of smooth muscle contraction [GO:0045986]; is part of GO:0042311 Also known as: relaxation of vascular smooth muscle, vascular smooth muscle relaxation, negative regulation of relaxation of vascular smooth muscle, positive regulation of relaxation of vascular smooth muscle, regulation of relaxation of vascular smooth muscle Definition: A negative regulation of smooth muscle contraction resulting in relaxation of vascular smooth muscle. The relaxation is mediated by a decrease in the phosphorylation state of myosin light chain. This can be achieved by removal of calcium from the cytoplasm to the sarcoplasmic reticulum lumen through the action of Ca2+ ATPases leading to a decrease myosin light chain kinase activity, and through calcium-independent pathways leading to a increase in myosin light chain phosphatase activity.